{
  "gene_symbol": "CSRP1",
  "term_id": "GO:0060537",
  "term_label": "muscle tissue development",
  "gene_name": "Cysteine and glycine-rich protein 1",
  "gene": "UniProtKB:P21291"
}